{
  "term_id": "UNKNOWN:0002",
  "term_label": "Unknown biological process",
  "gene_symbol": "PLEKHM3",
  "gene_name": "Pleckstrin homology domain-containing family M member 3",
  "gene": "UniProtKB:Q6ZWE6"
}